{
  "gene_symbol": "RORC",
  "term_id": "GO:0004879",
  "gene": "UniProtKB:P51449",
  "gene_name": "Nuclear receptor ROR-gamma",
  "term_label": "nuclear receptor activity"
}